methyl ethyl ketone catabolic process [GO:0046213] (biological process) Also known as: methyl ethyl ketone breakdown, methyl ethyl ketone catabolism, methyl ethyl ketone degradation Sources: GOC:ai Relationships: is a type of GO:0042178; is a type of GO:0042182 Definition: The chemical reactions and pathways resulting in the breakdown of methyl ethyl ketone, a clear, colorless liquid with a fragrant, mint-like odor.